{
  "term_id": "GO:0001725",
  "gene_symbol": "TRIP6",
  "term_label": "stress fiber",
  "gene": "UniProtKB:Q15654",
  "gene_name": "Thyroid receptor-interacting protein 6"
}